{
  "term_id": "GO:0003725",
  "gene_symbol": "ADAR",
  "gene": "UniProtKB:P55265",
  "term_label": "double-stranded RNA binding",
  "gene_name": "Double-stranded RNA-specific adenosine deaminase"
}